{
  "gene_name": "Fizzy-related protein homolog",
  "term_id": "GO:0031145",
  "gene": "UniProtKB:Q9UM11",
  "term_label": "anaphase-promoting complex-dependent catabolic process",
  "gene_symbol": "FZR1"
}